positive regulation of transcription by galactose [GO:0000411] (biological process) Definition: Any process involving galactose that activates or increases the rate of transcription. Also known as: up regulation of transcription by galactose, up-regulation of transcription by galactose, upregulation of transcription by galactose, activation of transcription by galactose, stimulation of transcription by galactose Subtypes: GO:0000435 Relationships: is a type of regulation of transcription by galactose [GO:0000409]; is a type of carbon catabolite activation of transcription [GO:0045991] Sources: GOC:go_curators